{
  "term_id": "GO:0031267",
  "term_label": "small GTPase binding",
  "gene_symbol": "RILPL1",
  "gene_name": "RILP-like protein 1",
  "gene": "UniProtKB:Q5EBL4"
}